phospholipase C-activating G protein-coupled receptor signaling pathway [GO:0007200] (biological process) Subtypes: GO:0007206, phospholipase C-activating G protein-coupled acetylcholine receptor signaling pathway [GO:0007207], GO:0007208, phospholipase C-activating tachykinin receptor signaling pathway [GO:0007209], phospholipase C-activating opsin-mediated signaling pathway [GO:0030265], phospholipase C-activating dopamine receptor signaling pathway [GO:0060158], phospholipase C-activating adrenergic receptor signaling pathway [GO:0071882], phospholipase C-activating angiotensin-activated signaling pathway [GO:0086097], phospholipase C-activating endothelin receptor signaling pathway [GO:0160135] Also known as: G protein signaling, coupled to IP3 second messenger (phospholipase C activating), G protein signalling, coupled to IP3 second messenger (phospholipase C activating), G-protein coupled receptor signaling pathway coupled to IP3 second messenger, G-protein signaling, coupled to IP3 second messenger (phospholipase C activating), G-protein signalling, coupled to IP3 second messenger (phospholipase C activating), PLC-activating GPCR signaling pathway, phospholipase C-activating G-protein coupled receptor signaling pathway, protein kinase C-activating G protein-coupled receptor signaling pathway, activation of phospholipase C activity by G-protein coupled receptor protein signaling pathway coupled to IP3 second messenger Sources: GOC:dph, GOC:mah, GOC:signaling, GOC:tb, ISBN:0815316194 Definition: A G protein-coupled receptor signaling pathway in which the signal is transmitted via the activation of phospholipase C (PLC) and a subsequent increase in the intracellular concentration of inositol trisphosphate (IP3) and diacylglycerol (DAG). IP3 regulates the opening of calcium channels in intracellular calcium store, leading to the release of calcium into the cytosol. Calcium and DAG activate protein kinase C (PKC), which in turn activates downstream effectors. Regulation: regulated by regulation of phospholipase C-activating G protein-coupled receptor signaling pathway [GO:1900736]; negatively regulated by negative regulation of phospholipase C-activating G protein-coupled receptor signaling pathway [GO:1900737]; positively regulated by GO:1900738 Relationships: is a type of G protein-coupled receptor signaling pathway [GO:0007186]; has part GO:0160185